interleukin-27 production [GO:0032631] (biological process) Definition: The appearance of interleukin-27 due to biosynthesis or secretion following a cellular stimulus, resulting in an increase in its intracellular or extracellular levels. Sources: GOC:mah Also known as: IL-27 production, interleukin-27 biosynthetic process, interleukin-27 formation, interleukin-27 secretion, interleukin-27 synthesis Relationships: is a type of GO:0001816 Regulation: regulated by GO:0032671; negatively regulated by negative regulation of interleukin-27 production [GO:0032711]; positively regulated by positive regulation of interleukin-27 production [GO:0032751]